{
  "gene_name": "Lysocardiolipin acyltransferase 1",
  "term_label": "endomembrane system",
  "gene_symbol": "LCLAT1",
  "gene": "UniProtKB:Q6UWP7",
  "term_id": "GO:0012505"
}